{
  "term_label": "cell adhesion",
  "term_id": "GO:0007155",
  "gene": "UniProtKB:P05362",
  "gene_symbol": "ICAM1",
  "gene_name": "Intercellular adhesion molecule 1"
}